negative regulation of mesenchymal stem cell migration [GO:1905321] (biological process) Definition: Any process that stops, prevents or reduces the frequency, rate or extent of mesenchymal stem cell migration. Also known as: down regulation of mesenchymal stem cell migration, down-regulation of mesenchymal stem cell migration, downregulation of mesenchymal stem cell migration, inhibition of mesenchymal stem cell migration References: PMID:26846297 Sources: GOC:TermGenie, GO_REF:0000058 Relationships: is a type of negative regulation of cell migration [GO:0030336]; is a type of GO:1905320; negatively regulates mesenchymal stem cell migration [GO:1905319]